{
  "term_label": "tissue regeneration",
  "term_id": "GO:0042246",
  "gene": "UniProtKB:P17677",
  "gene_symbol": "GAP43",
  "gene_name": "Neuromodulin"
}